{
  "gene_symbol": "AKR1C3",
  "term_id": "GO:0044597",
  "gene": "UniProtKB:P42330",
  "gene_name": "Aldo-keto reductase family 1 member C3",
  "term_label": "daunorubicin metabolic process"
}